fungal-type cell wall assembly [GO:0071940] (biological process) Subtypes: GO:0030476 References: PMID:19646873 Sources: GOC:mah, GOC:vw Relationships: is a type of GO:0031505; is a type of cell wall assembly [GO:0070726]; is part of fungal-type cell wall biogenesis [GO:0009272] Also known as: fungal-type cell wall formation Definition: The aggregation, arrangement and bonding together of a set of components to form a fungal-type cell wall.